{
  "term_id": "GO:1902476",
  "gene_symbol": "BEST3",
  "gene": "UniProtKB:Q8N1M1",
  "gene_name": "Bestrophin-3",
  "term_label": "chloride transmembrane transport"
}